{
  "term_id": "GO:0000981",
  "gene": "UniProtKB:Q13952",
  "term_label": "DNA-binding transcription factor activity, RNA polymerase II-specific",
  "gene_symbol": "NFYC",
  "gene_name": "Nuclear transcription factor Y subunit gamma"
}